{
  "gene_symbol": "ZNF33B",
  "gene_name": "Zinc finger protein 33B",
  "term_label": "transcription cis-regulatory region binding",
  "term_id": "GO:0000976",
  "gene": "UniProtKB:Q06732"
}